podocyte differentiation [GO:0072112] (biological process) Relationships: is a type of renal filtration cell differentiation [GO:0061318]; is a type of glomerular epithelial cell differentiation [GO:0072311] Definition: The process in which a relatively unspecialized cell acquires specialized features of a glomerular visceral epithelial cell. A glomerular visceral epithelial cell is a specialized epithelial cell that contains 'feet' that interdigitate with the 'feet' of other glomerular epithelial cells. Subtypes: mesonephric podocyte differentiation [GO:0061256], metanephric podocyte differentiation [GO:0072248] Also known as: glomerular visceral epithelial cell differentiation Sources: GOC:mtg_kidney_jan10